{
  "term_id": "UNKNOWN:0003",
  "gene_symbol": "ACYP1",
  "gene_name": "Acylphosphatase-1",
  "term_label": "Unknown cellular component",
  "gene": "UniProtKB:P07311"
}